{
  "term_id": "GO:0006511",
  "term_label": "ubiquitin-dependent protein catabolic process",
  "gene_symbol": "RNF14",
  "gene_name": "E3 ubiquitin-protein ligase RNF14",
  "gene": "UniProtKB:Q9UBS8"
}